{
  "term_id": "GO:0038203",
  "gene": "UniProtKB:Q96A49",
  "term_label": "TORC2 signaling",
  "gene_symbol": "SYAP1",
  "gene_name": "Synapse-associated protein 1"
}